{
  "gene": "UniProtKB:O95071",
  "gene_name": "E3 ubiquitin-protein ligase UBR5",
  "term_id": "GO:0090263",
  "term_label": "positive regulation of canonical Wnt signaling pathway",
  "gene_symbol": "UBR5"
}